sodium:iodide symporter activity [GO:0008507] (molecular function) Definition: Enables the transfer of a solute or solutes from one side of a membrane to the other according to the reaction: iodide(out) + Na+(out) = iodide(in) + Na+(in). Also known as: sodium/iodide symporter activity Relationships: is a type of GO:0015111; is a type of monoatomic anion:sodium symporter activity [GO:0015373] Sources: TC:2.A.21.5.1